UDP-galactose:glucosylceramide beta-1,4-galactosyltransferase activity [GO:0008489] (molecular function) Definition: Catalysis of the reaction: a beta-D-glucosyl-(1<->1')-N-acylsphing-4-enine + UDP-alpha-D-galactose = a beta-D-Gal-(1->4)-beta-D-Glc-(1<->1)-Cer(d18:1(4E)) + H+ + UDP. Relationships: is a type of UDP-galactosyltransferase activity [GO:0035250] References: PMID:9593693 Sources: RHEA:31495 Also known as: LacCer synthase activity, UDP-galactose glucosylceramide beta-1,4-galactosyltransferase activity, lactosylceramide synthase activity